{
  "gene_name": "Gap junction alpha-8 protein",
  "gene": "UniProtKB:P48165",
  "term_label": "connexin complex",
  "gene_symbol": "GJA8",
  "term_id": "GO:0005922"
}